{
  "term_label": "high-density lipoprotein particle clearance",
  "gene_name": "Apolipoprotein M",
  "gene": "UniProtKB:O95445",
  "term_id": "GO:0034384",
  "gene_symbol": "APOM"
}